{
  "term_id": "GO:0071805",
  "gene": "UniProtKB:Q12791",
  "gene_symbol": "KCNMA1",
  "term_label": "potassium ion transmembrane transport",
  "gene_name": "Calcium-activated potassium channel subunit alpha-1"
}